{
  "gene": "UniProtKB:P35998",
  "term_id": "GO:0036402",
  "gene_symbol": "PSMC2",
  "gene_name": "26S proteasome regulatory subunit 7",
  "term_label": "proteasome-activating activity"
}